acute inflammatory response [GO:0002526] (biological process) Relationships: is a type of inflammatory response [GO:0006954] Subtypes: GO:0002254, GO:0002438, acute inflammatory response to non-antigenic stimulus [GO:0002525], GO:0006953, resolution phase response [GO:0106299] Definition: Inflammation which comprises a rapid, short-lived, relatively uniform response to acute injury or antigenic challenge and is characterized by accumulations of fluid, plasma proteins, and granulocytic leukocytes. An acute inflammatory response occurs within a matter of minutes or hours, and either resolves within a few days or becomes a chronic inflammatory response. Sources: GOC:add, GO_REF:0000022, ISBN:0781735149 Regulation: regulated by regulation of acute inflammatory response [GO:0002673]; negatively regulated by negative regulation of acute inflammatory response [GO:0002674]; positively regulated by positive regulation of acute inflammatory response [GO:0002675]